{
  "gene_symbol": "PSMC3IP",
  "term_label": "meiotic joint molecule formation",
  "term_id": "GO:0000709",
  "gene": "UniProtKB:Q9P2W1",
  "gene_name": "Homologous-pairing protein 2 homolog"
}